{
  "term_label": "regulation of endocytosis",
  "gene_symbol": "ARFGAP1",
  "gene": "UniProtKB:Q8N6T3",
  "gene_name": "ADP-ribosylation factor GTPase-activating protein 1",
  "term_id": "GO:0030100"
}